{
  "gene": "UniProtKB:A0A5B7",
  "gene_symbol": "TRBV29-1",
  "term_id": "GO:0007166",
  "term_label": "cell surface receptor signaling pathway",
  "gene_name": "T cell receptor beta variable 29-1"
}